{
  "gene_symbol": "NPEPL1",
  "term_label": "cytoplasm",
  "gene_name": "Probable aminopeptidase NPEPL1",
  "term_id": "GO:0005737",
  "gene": "UniProtKB:Q8NDH3"
}